positive regulation of substrate-dependent cell migration, cell attachment to substrate [GO:1904237] (biological process) Also known as: positive regulation of substrate-bound cell migration, cell attachment to substrate, up regulation of substrate-bound cell migration, cell attachment to substrate, up regulation of substrate-dependent cell migration, cell attachment to substrate, up-regulation of substrate-bound cell migration, cell attachment to substrate, up-regulation of substrate-dependent cell migration, cell attachment to substrate, upregulation of substrate-bound cell migration, cell attachment to substrate, upregulation of substrate-dependent cell migration, cell attachment to substrate, activation of substrate-bound cell migration, cell attachment to substrate, activation of substrate-dependent cell migration, cell attachment to substrate References: PMID:25834989 Sources: GOC:TermGenie, GO_REF:0000058 Definition: Any process that activates or increases the frequency, rate or extent of substrate-dependent cell migration, cell attachment to substrate. Relationships: is a type of positive regulation of cell-substrate adhesion [GO:0010811]; is a type of positive regulation of cell migration [GO:0030335]; is a type of GO:1904235; positively regulates GO:0006931